{
  "term_label": "pentameric IgM immunoglobulin complex",
  "gene": "UniProtKB:P01591",
  "gene_name": "Immunoglobulin J chain",
  "term_id": "GO:0071756",
  "gene_symbol": "JCHAIN"
}